{
  "gene_symbol": "SSUH2",
  "term_id": "UNKNOWN:0002",
  "term_label": "Unknown biological process",
  "gene_name": "Protein SSUH2 homolog",
  "gene": "UniProtKB:Q9Y2M2"
}